{
  "term_id": "GO:0048240",
  "gene_symbol": "EFCAB9",
  "gene_name": "EF-hand calcium-binding domain-containing protein 9",
  "gene": "UniProtKB:A8MZ26",
  "term_label": "sperm capacitation"
}